{
  "term_label": "RNA polymerase II cis-regulatory region sequence-specific DNA binding",
  "gene": "UniProtKB:Q14585",
  "gene_name": "Zinc finger protein 345",
  "gene_symbol": "ZNF345",
  "term_id": "GO:0000978"
}